aspartic endopeptidase activity, intramembrane cleaving [GO:0042500] (molecular function) Note: Note that although GO generally avoids the use of localization information in terms, in this case an exception was made. This is because the fact that the cleavage occurs within the membrane is integral to its function, as it is the only thing that distinguishes this group from other aspartic endopeptidases. Sources: GOC:jl, ISBN:0198506732 Relationships: is a type of GO:0004190 Definition: Catalysis of the hydrolysis of nonterminal peptide bonds in a polypeptide chain, occurring within a membrane.